{
  "gene_name": "Dynein axonemal heavy chain 11",
  "gene": "UniProtKB:Q96DT5",
  "term_label": "dynein light intermediate chain binding",
  "term_id": "GO:0051959",
  "gene_symbol": "DNAH11"
}